{
  "gene": "UniProtKB:Q96FZ5",
  "term_id": "UNKNOWN:0002",
  "term_label": "Unknown biological process",
  "gene_symbol": "CMTM7",
  "gene_name": "CKLF-like MARVEL transmembrane domain-containing protein 7"
}